{
  "term_label": "Unknown biological process",
  "gene": "UniProtKB:Q68EN5",
  "gene_name": "Microtubule-associated tyrosine carboxypeptidase 1",
  "term_id": "UNKNOWN:0002",
  "gene_symbol": "MATCAP1"
}